{
  "gene_symbol": "RNF24",
  "gene_name": "RING finger protein 24",
  "term_label": "Unknown molecular function",
  "gene": "UniProtKB:Q9Y225",
  "term_id": "UNKNOWN:0001"
}